{
  "gene": "UniProtKB:P23443",
  "term_label": "TORC1 signaling",
  "gene_name": "Ribosomal protein S6 kinase beta-1",
  "term_id": "GO:0038202",
  "gene_symbol": "RPS6KB1"
}